{
  "gene_name": "Suppressor of cytokine signaling 2",
  "term_id": "GO:0046426",
  "term_label": "negative regulation of receptor signaling pathway via JAK-STAT",
  "gene_symbol": "SOCS2",
  "gene": "UniProtKB:O14508"
}